{
  "gene_name": "Importin subunit alpha-8",
  "gene_symbol": "KPNA7",
  "term_label": "nuclear import signal receptor activity",
  "term_id": "GO:0061608",
  "gene": "UniProtKB:A9QM74"
}